forebrain-midbrain boundary formation [GO:0021905] (biological process) References: PMID:11262869 Sources: GOC:cls, GOC:dgh, GOC:dph, GOC:jid, GO_REF:0000021 Definition: The process whose specific outcome is the creation of the forebrain-midbrain boundary. Relationships: is_a anatomical structure development [GO:0048856]; is a type of formation of anatomical boundary [GO:0048859]; is part of rostrocaudal neural tube patterning [GO:0021903]